{
  "gene": "UniProtKB:P55283",
  "gene_symbol": "CDH4",
  "gene_name": "Cadherin-4",
  "term_label": "cell-cell adhesion mediated by cadherin",
  "term_id": "GO:0044331"
}